{
  "gene_symbol": "VAT1",
  "gene_name": "Synaptic vesicle membrane protein VAT-1 homolog",
  "term_label": "mitochondrial outer membrane",
  "gene": "UniProtKB:Q99536",
  "term_id": "GO:0005741"
}